{
  "term_label": "negative regulation of transcription by RNA polymerase II",
  "gene_name": "Zinc finger protein ZFPM2",
  "term_id": "GO:0000122",
  "gene": "UniProtKB:Q8WW38",
  "gene_symbol": "ZFPM2"
}